negative regulation of protein localization to adherens junction [GO:1904703] (BP) Relationships: is a type of GO:0150119; is a type of GO:1904702; negatively regulates protein localization to adherens junction [GO:0071896] Also known as: down regulation of protein localisation in cell-cell adherens junction, down regulation of protein localisation to cell-cell adherens junction, down regulation of protein localization in cell-cell adherens junction, down regulation of protein localization to cell-cell adherens junction, down-regulation of protein localisation in cell-cell adherens junction, down-regulation of protein localisation to cell-cell adherens junction, down-regulation of protein localization in cell-cell adherens junction, down-regulation of protein localization to cell-cell adherens junction, downregulation of protein localisation in cell-cell adherens junction, downregulation of protein localisation to cell-cell adherens junction, downregulation of protein localization in cell-cell adherens junction, downregulation of protein localization to cell-cell adherens junction, negative regulation of protein localisation in cell-cell adherens junction, negative regulation of protein localisation to cell-cell adherens junction, negative regulation of protein localization in cell-cell adherens junction, inhibition of protein localisation in cell-cell adherens junction, inhibition of protein localisation to cell-cell adherens junction, inhibition of protein localization in cell-cell adherens junction, inhibition of protein localization to cell-cell adherens junction References: PMID:26412237 Sources: GOC:TermGenie, GOC:aruk, GOC:bc, GOC:kmv, GO_REF:0000058 Definition: Any process that stops, prevents or reduces the frequency, rate or extent of protein localization to adherens junction. An adherens junction is a cell-cell junction composed of the epithelial cadherin-catenin complex at which the cytoplasmic face of the plasma membrane is attached to actin filaments.